{
  "gene_symbol": "GOLGA6L26",
  "term_label": "Unknown biological process",
  "term_id": "UNKNOWN:0002",
  "gene_name": "Golgin subfamily A member 6-like protein 26",
  "gene": "UniProtKB:P0DX02"
}